{
  "term_id": "GO:0070306",
  "gene_symbol": "MAF",
  "gene_name": "Transcription factor Maf",
  "gene": "UniProtKB:O75444",
  "term_label": "lens fiber cell differentiation"
}